{
  "gene_symbol": "APOO",
  "term_id": "GO:0042407",
  "gene": "UniProtKB:Q9BUR5",
  "gene_name": "MICOS complex subunit MIC26",
  "term_label": "cristae formation"
}